{
  "gene": "UniProtKB:P86434",
  "term_label": "Unknown molecular function",
  "gene_name": "Putative uncharacterized protein ADORA2A-AS1",
  "gene_symbol": "ADORA2A-AS1",
  "term_id": "UNKNOWN:0001"
}